{
  "term_id": "GO:0005886",
  "gene_name": "Glutamate receptor ionotropic, kainate 5",
  "gene": "UniProtKB:Q16478",
  "gene_symbol": "GRIK5",
  "term_label": "plasma membrane"
}